{
  "gene_symbol": "POLD3",
  "term_id": "GO:0003887",
  "term_label": "DNA-directed DNA polymerase activity",
  "gene_name": "DNA polymerase delta subunit 3",
  "gene": "UniProtKB:Q15054"
}